{
  "term_id": "GO:0043484",
  "term_label": "regulation of RNA splicing",
  "gene_symbol": "HNRNPH2",
  "gene": "UniProtKB:P55795",
  "gene_name": "Heterogeneous nuclear ribonucleoprotein H2"
}